{
  "term_id": "GO:0000122",
  "gene": "UniProtKB:Q86UQ0",
  "gene_symbol": "ZNF589",
  "gene_name": "Zinc finger protein 589",
  "term_label": "negative regulation of transcription by RNA polymerase II"
}